{
  "term_id": "GO:0045892",
  "gene_symbol": "SBNO2",
  "gene_name": "Protein strawberry notch homolog 2",
  "term_label": "negative regulation of DNA-templated transcription",
  "gene": "UniProtKB:Q9Y2G9"
}